regulation of copper ion transmembrane transport [GO:1902311] (biological process) Definition: Any process that modulates the frequency, rate or extent of copper ion transmembrane transport. Also known as: regulation of copper cation transmembrane transport, regulation of copper ion membrane transport References: PMID:21489137 Sources: GOC:TermGenie, GOC:di Relationships: is a type of regulation of metal ion transport [GO:0010959]; is a type of GO:1904062; regulates copper ion transmembrane transport [GO:0035434] Subtypes: negative regulation of copper ion transmembrane transport [GO:1902312], positive regulation of copper ion transmembrane transport [GO:1902313]